{
  "term_label": "nucleus",
  "gene": "UniProtKB:Q9NP08",
  "gene_symbol": "HMX1",
  "term_id": "GO:0005634",
  "gene_name": "Homeobox protein HMX1"
}